{
  "gene_symbol": "FAM107A",
  "gene": "UniProtKB:O95990",
  "term_id": "GO:0032956",
  "term_label": "regulation of actin cytoskeleton organization",
  "gene_name": "Actin-associated protein FAM107A"
}